{
  "gene_symbol": "SERPINB1",
  "gene_name": "Leukocyte elastase inhibitor",
  "term_id": "GO:0004867",
  "term_label": "serine-type endopeptidase inhibitor activity",
  "gene": "UniProtKB:P30740"
}